{
  "gene_symbol": "APOC3",
  "gene_name": "Apolipoprotein C-III",
  "gene": "UniProtKB:P02656",
  "term_id": "GO:0010989",
  "term_label": "negative regulation of low-density lipoprotein particle clearance"
}